{
  "term_label": "regulation of skeletal muscle contraction by regulation of release of sequestered calcium ion",
  "gene": "UniProtKB:P31415",
  "gene_name": "Calsequestrin-1",
  "gene_symbol": "CASQ1",
  "term_id": "GO:0014809"
}